{
  "gene_symbol": "RHD",
  "term_label": "plasma membrane",
  "gene_name": "Blood group Rh(D) polypeptide",
  "gene": "UniProtKB:Q02161",
  "term_id": "GO:0005886"
}